{
  "term_id": "UNKNOWN:0001",
  "term_label": "Unknown molecular function",
  "gene_name": "Transmembrane protein 174",
  "gene": "UniProtKB:Q8WUU8",
  "gene_symbol": "TMEM174"
}